DNA recombinase mediator complex [GO:0033061] (CC) Subtypes: GO:0032798, Rad51B-Rad51C-Rad51D-XRCC2 complex [GO:0033063], XRCC2-RAD51D complex [GO:0033064], GO:0033065, Rad51B-Rad51C complex [GO:0033066] Relationships: is a type of protein-containing complex [GO:0032991] References: PMID:12912992, PMID:32414915 Sources: GOC:elh, GOC:mah, GOC:vw, InterPro:IPR003488 Note: Many paralogs of Rad51 act as recombinase mediators. These paralogs dimerize (or occasionally form tetramers) amongst themselves to form complexes with ssDNA-binding activity, and which act as mediators of Rad51 presynaptic filament assembly. Definition: A protein complex containing accessory proteins which bind a recombinase (e.g. Rad51) and bind single-stranded DNA (ssDNA), and promote nucleation of the recombinase onto ssDNA through facilitating recombinase-RPA exchange.